{
  "gene": "UniProtKB:Q92564",
  "gene_symbol": "DCUN1D4",
  "term_id": "GO:0031624",
  "gene_name": "DCN1-like protein 4",
  "term_label": "ubiquitin conjugating enzyme binding"
}